{
  "gene": "UniProtKB:Q96N66",
  "gene_symbol": "MBOAT7",
  "term_id": "GO:0044233",
  "gene_name": "Lysophospholipid acyltransferase 7",
  "term_label": "mitochondria-associated endoplasmic reticulum membrane contact site"
}